{
  "gene_name": "Non-homologous end-joining factor 1",
  "gene_symbol": "NHEJ1",
  "term_label": "double-strand break repair via nonhomologous end joining",
  "gene": "UniProtKB:Q9H9Q4",
  "term_id": "GO:0006303"
}